mitotic sister chromatid segregation [GO:0000070] (biological process) Also known as: mitotic chromosome segregation, mitotic sister-chromatid adhesion release Definition: The cell cycle process in which replicated homologous chromosomes are organized and then physically separated and apportioned to two sets during the mitotic cell cycle. Each replicated chromosome, composed of two sister chromatids, aligns at the cell equator, paired with its homologous partner. One homolog of each morphologic type goes into each of the resulting chromosome sets. Relationships: is a type of sister chromatid segregation [GO:0000819]; is a type of mitotic cell cycle process [GO:1903047]; is part of mitotic nuclear division [GO:0140014] Sources: GOC:ai, GOC:jl Regulation: regulated by regulation of mitotic sister chromatid segregation [GO:0033047]; RO_0002212 by negative regulation of mitotic sister chromatid segregation [GO:0033048]; positively regulated by positive regulation of mitotic sister chromatid segregation [GO:0062033]